{
  "term_id": "GO:0050911",
  "term_label": "detection of chemical stimulus involved in sensory perception of smell",
  "gene_name": "Olfactory receptor 10Z1",
  "gene": "UniProtKB:Q8NGY1",
  "gene_symbol": "OR10Z1"
}